{
  "gene": "UniProtKB:O75390",
  "term_label": "mitochondrial matrix",
  "gene_name": "Citrate synthase, mitochondrial",
  "gene_symbol": "CS",
  "term_id": "GO:0005759"
}